{
  "gene_name": "Rap guanine nucleotide exchange factor 6",
  "gene_symbol": "RAPGEF6",
  "gene": "UniProtKB:Q8TEU7",
  "term_id": "GO:0007265",
  "term_label": "Ras protein signal transduction"
}